positive regulation of extracellular matrix organization [GO:1903055] (biological process) Relationships: is a type of positive regulation of cellular component organization [GO:0051130]; is a type of GO:1903053; positively regulates extracellular matrix organization [GO:0030198] References: PMID:22357537 Sources: GOC:BHF, GOC:TermGenie, GOC:rl, GO_REF:0000058 Also known as: positive regulation of extracellular matrix organisation, up regulation of extracellular matrix organisation, up regulation of extracellular matrix organization, up-regulation of extracellular matrix organisation, up-regulation of extracellular matrix organization, upregulation of extracellular matrix organisation, upregulation of extracellular matrix organization, activation of extracellular matrix organisation, activation of extracellular matrix organization, activation of extracellular matrix organization and biogenesis, positive regulation of extracellular matrix organization and biogenesis, up regulation of extracellular matrix organization and biogenesis, up-regulation of extracellular matrix organization and biogenesis, upregulation of extracellular matrix organization and biogenesis Definition: Any process that activates or increases the frequency, rate or extent of extracellular matrix organization. Subtypes: positive regulation of extracellular matrix constituent secretion [GO:0003331], positive regulation of extracellular matrix disassembly [GO:0090091], GO:1901203, positive regulation of collagen fibril organization [GO:1904028]